{
  "term_id": "GO:1990756",
  "gene_symbol": "CCIN",
  "term_label": "ubiquitin-like ligase-substrate adaptor activity",
  "gene_name": "Calicin",
  "gene": "UniProtKB:Q13939"
}